{
  "gene_symbol": "UGT1A5",
  "gene_name": "UDP-glucuronosyltransferase 1A5",
  "term_label": "flavone metabolic process",
  "term_id": "GO:0051552",
  "gene": "UniProtKB:P35504"
}